regulation of cell-substrate junction assembly [GO:0090109] (biological process) Sources: GOC:dph, GOC:tb Definition: Any process that modulates the rate, frequency, or extent of cell-substrate junction assembly. Cell-substrate junction assembly is the aggregation, arrangement and bonding together of a set of components to form a junction between a cell and its substrate. Subtypes: regulation of focal adhesion assembly [GO:0051893] Relationships: is a type of GO:0150116; is_a regulation of cell junction assembly [GO:1901888]; regulates cell-substrate junction assembly [GO:0007044]